{
  "gene_symbol": "HSH2D",
  "gene_name": "Hematopoietic SH2 domain-containing protein",
  "term_id": "GO:0042110",
  "gene": "UniProtKB:Q96JZ2",
  "term_label": "T cell activation"
}